mitochondrial tRNA 5'-end processing [GO:0097745] (biological process) Relationships: is_a mitochondrial RNA 5'-end processing [GO:0000964]; is a type of GO:0090646; is_a tRNA 5'-end processing [GO:0099116] Definition: The process in which the 5' end of a pre-tRNA molecule is converted to that of a mature tRNA in the mitochondrion. References: PMID:21307182, PMID:26143376, PMID:27484477 Sources: GOC:pf